{
  "gene": "UniProtKB:Q5T9A4",
  "gene_symbol": "ATAD3B",
  "term_id": "GO:0007005",
  "term_label": "mitochondrion organization",
  "gene_name": "ATPase family AAA domain-containing protein 3B"
}